{
  "term_label": "positive regulation of phagocytosis",
  "term_id": "GO:0050766",
  "gene": "UniProtKB:Q9P1W8",
  "gene_symbol": "SIRPG",
  "gene_name": "Signal-regulatory protein gamma"
}